SNARE binding [GO:0000149] (molecular function) Definition: Binding to a SNARE (soluble N-ethylmaleimide-sensitive factor attached protein receptor) protein. Also known as: SNAP receptor binding References: PMID:12642621 Subtypes: syntaxin binding [GO:0019905] Relationships: is a type of protein binding [GO:0005515]